histone deubiquitinase activity [GO:0140934] (molecular function) References: PMID:18206972, PMID:18226187 Definition: A deubiquitinase that cleaves ubiquitin from a histone protein to which it is conjugated. Relationships: is a type of GO:0101005; is a type of histone modifying activity [GO:0140993] Subtypes: histone H2B deubiquitinase activity [GO:0140936], GO:0140950 Also known as: histone deubiquitination